{
  "gene": "UniProtKB:Q6ZUT9",
  "gene_symbol": "DENND5B",
  "gene_name": "DENN domain-containing protein 5B",
  "term_label": "small GTPase binding",
  "term_id": "GO:0031267"
}